{
  "term_id": "UNKNOWN:0002",
  "gene": "UniProtKB:O75425",
  "gene_name": "Motile sperm domain-containing protein 3",
  "gene_symbol": "MOSPD3",
  "term_label": "Unknown biological process"
}